response to lipopolysaccharide [GO:0032496] (biological process) Sources: GOC:add, ISBN:0721601464 Also known as: response to endotoxin, response to LPS Relationships: is a type of GO:0002237; is a type of response to lipid [GO:0033993]; is a type of response to oxygen-containing compound [GO:1901700] Definition: Any process that results in a change in state or activity of an organism (in terms of movement, secretion, enzyme production, gene expression, etc.) as a result of a lipopolysaccharide stimulus; lipopolysaccharide is a major component of the cell wall of gram-negative bacteria. Subtypes: detection of lipopolysaccharide [GO:0032497], cellular response to lipopolysaccharide [GO:0071222]